{
  "gene_name": "Olfactory receptor 8A1",
  "term_label": "sensory perception of smell",
  "term_id": "GO:0007608",
  "gene": "UniProtKB:Q8NGG7",
  "gene_symbol": "OR8A1"
}